{
  "gene_symbol": "TNFRSF1A",
  "gene_name": "Tumor necrosis factor receptor superfamily member 1A",
  "term_label": "membrane raft",
  "gene": "UniProtKB:P19438",
  "term_id": "GO:0045121"
}